extrachromosomal DNA [GO:0046821] (cellular component) Definition: DNA structures that are not part of a chromosome. Relationships: is a type of intracellular anatomical structure [GO:0005622] Sources: GOC:ai